L-methionine salvage from methylthioadenosine [GO:0019509] (biological process) Also known as: methionine salvage from methylthioadenosine, methionine salvage pathway, methionine recycling, methionine regeneration Definition: The generation of L-methionine (2-amino-4-(methylthio)butanoic acid) from methylthioadenosine. References: PMID:19946895 Sources: GOC:jl, MetaCyc:PWY-4361 Relationships: is a type of GO:0071267